{
  "gene": "UniProtKB:Q8WXU2",
  "term_label": "heart development",
  "gene_name": "Dynein axonemal assembly factor 4",
  "term_id": "GO:0007507",
  "gene_symbol": "DNAAF4"
}